dIDP phosphatase activity [GO:0097383] (molecular function) References: PMID:20385596 Sources: GOC:pde, RHEA:35211 Definition: Catalysis of the reaction: dIDP + H2O = dIMP + H+ + phosphate. Also known as: deoxyinosine-diphosphatase activity Relationships: is_a GO:0017110